{
  "gene_symbol": "RRM2B",
  "gene": "UniProtKB:Q7LG56",
  "gene_name": "Ribonucleoside-diphosphate reductase subunit M2 B",
  "term_id": "GO:0009263",
  "term_label": "deoxyribonucleotide biosynthetic process"
}